cellular process [GO:0009987] (biological process) Also known as: cell physiology, cellular physiological process, cell growth and/or maintenance, single-organism cellular process Subtypes: septum digestion after cytokinesis [GO:0000920], cell activation [GO:0001775], cell killing [GO:0001906], plasmid maintenance [GO:0006276], GO:0006457, vesicle targeting [GO:0006903], GO:0006949, microtubule-based process [GO:0007017], cell cycle [GO:0007049], cell communication [GO:0007154], cell adhesion [GO:0007155], GO:0007163, GO:0007165, GO:0007272, GO:0008037, metabolic process [GO:0008152], cell death [GO:0008219], GO:0008283, horizontal gene transfer [GO:0009292], GO:0010118, intercellular transport [GO:0010496], light absorption [GO:0016037], cell growth [GO:0016049], vesicle-mediated transport [GO:0016192], cytolysis [GO:0019835], cell cycle process [GO:0022402], GO:0022406, cellular process involved in reproduction in multicellular organism [GO:0022412], actin filament-based process [GO:0030029], transposition [GO:0032196], cellular pigmentation [GO:0033059], GO:0034337, cell competition in a multicellular organism [GO:0035212], phenotypic switching [GO:0036166], protein unfolding [GO:0043335], establishment or maintenance of cell type involved in phenotypic switching [GO:0044663], intermediate filament-based process [GO:0045103], GO:0048489, GO:0048869, GO:0048870, cell division [GO:0051301], cellular localization [GO:0051641], GO:0051651, localization of cell [GO:0051674], cellular response to stimulus [GO:0051716], transmembrane transport [GO:0055085], cell adhesion molecule production [GO:0060352], microtubule organizing center localization [GO:0061842], process utilizing autophagic mechanism [GO:0061919], cell wall organization or biogenesis [GO:0071554], GO:0071840, cellular senescence [GO:0090398], GO:0097194, execution phase of necroptosis [GO:0097528], cell aggregation [GO:0098743], ciliary basal body segregation [GO:0120312], exocytic process [GO:0140029], cell-cell fusion [GO:0140253], export from cell [GO:0140352], nutrient storage [GO:0170062], cellular detoxification [GO:1990748] Note: This term should not be used for direct annotation. It should be possible to make a more specific annotation to one of the children of this term. Sources: GOC:go_curators, GOC:isa_complete Relationships: is_a biological_process [GO:0008150] Regulation: positively regulated by GO:0048522; negatively regulated by negative regulation of cellular process [GO:0048523]; RO_0002211 by GO:0050794 Definition: Any process that is carried out at the cellular level, but not necessarily restricted to a single cell. For example, cell communication occurs among more than one cell, but occurs at the cellular level.